{
  "gene": "UniProtKB:Q86XA0",
  "gene_symbol": "METTL23",
  "term_id": "GO:0035642",
  "term_label": "histone H3R17 methyltransferase activity",
  "gene_name": "Histone-arginine methyltransferase METTL23"
}